trans-synaptic signaling, modulating synaptic transmission [GO:0099550] (biological process) Definition: Cell-cell signaling between presynapse and postsynapse, across the synaptic cleft, that modulates the synaptic transmission properties of the synapse. Sources: GOC:dos Relationships: is a type of modulation of chemical synaptic transmission [GO:0050804]; is a type of trans-synaptic signaling [GO:0099537] Note: Note that this term was created for the SynGO project, and will be obsoleted when the SynGO annotations are made in Noctua. Subtypes: trans-synaptic signaling by BDNF, modulating synaptic transmission [GO:0099183], trans-synaptic signaling by neuropeptide, modulating synaptic transmission [GO:0099551], trans-synaptic signaling by lipid, modulating synaptic transmission [GO:0099552], trans-synaptic signaling by soluble gas, modulating synaptic transmission [GO:0099554], GO:0099557